{
  "gene_name": "Zinc finger protein 394",
  "term_label": "RNA polymerase II cis-regulatory region sequence-specific DNA binding",
  "gene": "UniProtKB:Q53GI3",
  "gene_symbol": "ZNF394",
  "term_id": "GO:0000978"
}